G-protein alpha(13)-synembrin complex [GO:0071155] (cellular component) References: PMID:12509430 Sources: GOC:mah Also known as: Ric-8A G alpha 13 subunit complex Relationships: is_a intracellular protein-containing complex [GO:0140535] Definition: A protein complex formed by the association of the guanine nucleotide exchange factor synembrin with the alpha(13) subunit of a heterotrimeric G protein.